abscisic acid-activated signaling pathway [GO:0009738] (biological process) Subtypes: abscisic acid-activated signaling pathway involved in stomatal movement [GO:1901527] References: PMID:24269821 Sources: GOC:signaling, GOC:sm Definition: The series of molecular signals generated by the binding of the plant hormone abscisic acid (ABA) to a receptor, and ending with modulation of a cellular process, e.g. transcription. Also known as: ABA signal transduction, ABA signaling, abscisic acid mediated signalling, abscisic acid signal transduction, abscisic acid-mediated signaling pathway Relationships: is_a hormone-mediated signaling pathway [GO:0009755]; is part of cellular response to abscisic acid stimulus [GO:0071215] Regulation: regulated by regulation of abscisic acid-activated signaling pathway [GO:0009787]; RO_0002212 by negative regulation of abscisic acid-activated signaling pathway [GO:0009788]; RO_0002213 by positive regulation of abscisic acid-activated signaling pathway [GO:0009789]